{
  "gene_name": "C2 calcium-dependent domain-containing protein 4A",
  "gene_symbol": "C2CD4A",
  "term_label": "Unknown biological process",
  "term_id": "UNKNOWN:0002",
  "gene": "UniProtKB:Q8NCU7"
}